{
  "gene_symbol": "TIFA",
  "term_id": "GO:0002753",
  "term_label": "cytoplasmic pattern recognition receptor signaling pathway",
  "gene": "UniProtKB:Q96CG3",
  "gene_name": "TRAF-interacting protein with FHA domain-containing protein A"
}